{
  "term_id": "GO:0005737",
  "gene": "UniProtKB:Q9HAU5",
  "gene_name": "Regulator of nonsense transcripts 2",
  "gene_symbol": "UPF2",
  "term_label": "cytoplasm"
}